flavin prenyltransferase activity [GO:0106141] (MF) Definition: Catalysis of the reaction: dimethylallyl phosphate + FMNH2 = phosphate + prenyl-FMNH2. Relationships: is a type of GO:0004659 References: PMID:26083743 Sources: RHEA:37743